{
  "term_label": "D-ribulose-phosphate 3-epimerase activity",
  "term_id": "GO:0004750",
  "gene_name": "Ribulose-phosphate 3-epimerase-like protein 1",
  "gene": "UniProtKB:Q2QD12",
  "gene_symbol": "RPEL1"
}